multicellular organismal-level iron ion homeostasis [GO:0060586] (biological process) Relationships: is a type of monoatomic cation homeostasis [GO:0055080]; is a type of inorganic ion homeostasis [GO:0098771]; is a type of GO:0140962 Definition: A chemical homeostatic process involved in the maintenance of a steady state level of iron within extracellular body fluids, such as blood, xylem or phloem, of a multicellular organism. This is distinct from maintenance of cellular homeostasis, which occurs within a cell. References: PMID:31431773 Also known as: multicellular organismal iron ion homeostasis